{
  "term_id": "GO:0005773",
  "gene": "UniProtKB:Q8NCI6",
  "gene_symbol": "GLB1L3",
  "term_label": "vacuole",
  "gene_name": "Beta-galactosidase-1-like protein 3"
}